cellular pigmentation [GO:0033059] (biological process) Subtypes: GO:0043482 Definition: The deposition or aggregation of coloring matter in a cell. Relationships: is a type of cellular process [GO:0009987]; is_a pigmentation [GO:0043473] Sources: GOC:mtg_MIT_16mar07